{
  "gene": "UniProtKB:Q9HC62",
  "term_label": "protein desumoylation",
  "gene_symbol": "SENP2",
  "term_id": "GO:0016926",
  "gene_name": "Sentrin-specific protease 2"
}